prolyl-tRNA aminoacylation [GO:0006433] (biological process) Definition: The process of coupling proline to prolyl-tRNA, catalyzed by prolyl-tRNA synthetase. The prolyl-tRNA synthetase is a class-II synthetase. The activated amino acid is transferred to the 3'-OH group of a methionine-accetping tRNA. Sources: GOC:mah, ISBN:0716730510 Relationships: is_a GO:0006418 Subtypes: mitochondrial prolyl-tRNA aminoacylation [GO:0070157]